{
  "term_label": "synaptic vesicle priming",
  "gene_symbol": "SV2A",
  "gene_name": "Synaptic vesicle glycoprotein 2A",
  "term_id": "GO:0016082",
  "gene": "UniProtKB:Q7L0J3"
}